negative regulation of phospholipase C-activating phototransduction signaling pathway [GO:0016060] (biological process) References: PMID:8316831 Sources: GOC:hb Also known as: metarhodopsin inactivation Definition: Any process that stops, prevents or reduces the frequency, rate or extent of phospholipase C-activating phototransduction signaling pathway. Activated rhodopsin (R*) is inactivated by a two-step process: first, R* is phosphorylated by rhodopsin kinase which lowers the activity of R*. Second, the protein arrestin binds to phosphorylated R* to de-activate it. Relationships: is a type of negative regulation of opsin-mediated signaling pathway [GO:0016059]; is a type of negative regulation of phospholipase C-activating G protein-coupled receptor signaling pathway [GO:1900737]; negatively regulates GO:0030265